{
  "term_label": "positive regulation of transcription by RNA polymerase II",
  "gene_symbol": "PPARD",
  "term_id": "GO:0045944",
  "gene_name": "Peroxisome proliferator-activated receptor delta",
  "gene": "UniProtKB:Q03181"
}